xanthine hydrolase activity [GO:0043836] (molecular function) Definition: Catalysis of the reaction: xanthine + H2O = 4-ureido-5-imidazole carboxylate. Relationships: is a type of hydrolase activity, acting on carbon-nitrogen (but not peptide) bonds, in cyclic amides [GO:0016812] Also known as: xanthinase activity References: PMID:13278326 Sources: MetaCyc:R127-RXN